{
  "gene_symbol": "RAB23",
  "term_label": "GTPase activity",
  "term_id": "GO:0003924",
  "gene": "UniProtKB:Q9ULC3",
  "gene_name": "Ras-related protein Rab-23"
}